{
  "gene_symbol": "CATSPER1",
  "gene": "UniProtKB:Q8NEC5",
  "term_id": "GO:0007283",
  "gene_name": "Cation channel sperm-associated protein 1",
  "term_label": "spermatogenesis"
}